peptide secretion, neurotransmission [GO:0061544] (biological process) Subtypes: GO:0061585 Relationships: is_a peptide secretion [GO:0002790]; is a type of GO:0007269 Sources: GOC:dph Definition: The controlled release of a peptide from a cell in which the peptide acts as a neurotransmitter.